{
  "term_label": "extraction of mislocalized protein from ER membrane",
  "gene_name": "Endoplasmic reticulum transmembrane helix translocase",
  "term_id": "GO:0140569",
  "gene_symbol": "ATP13A1",
  "gene": "UniProtKB:Q9HD20"
}